zinc ion import into endoplasmic reticulum [GO:0140209] (biological process) Definition: The directed import of zinc(2+) from the cytosol, across the endoplasmic reticulum membrane, into the endoplasmic reticulum. References: PMID:11886869, PMID:29529046 Relationships: is a type of cytosol to endoplasmic reticulum transport [GO:0046967]; is a type of zinc ion import into organelle [GO:0062111] Also known as: zinc ion import across endoplasmic reticulum, zinc ion import into ER, zinc(2+) import across endoplasmic reticulum, zinc(2+) import into endoplasmic reticulum Note: This term covers zinc(2+) import *across* the endoplasmic reticulum membrane through a channel or pore. It does not cover import via vesicle fusion with endoplasmic reticulum membrane, as in this case transport does not involve crossing the membrane.